{
  "gene": "UniProtKB:Q96P67",
  "gene_name": "Probable G-protein coupled receptor 82",
  "gene_symbol": "GPR82",
  "term_label": "Unknown cellular component",
  "term_id": "UNKNOWN:0003"
}